L-arginine conjugated cholate hydrolase activity [GO:7770007] (molecular function) Relationships: is a type of amino acid conjugated cholate hydrolase activity [GO:7770003] References: PMID:38326608 Sources: RHEA:79111 Definition: Catalysis of the reaction: cholate + L-arginine = L-arginocholate + H2O.